{
  "term_id": "UNKNOWN:0001",
  "term_label": "Unknown molecular function",
  "gene_symbol": "SSX3",
  "gene": "UniProtKB:Q99909",
  "gene_name": "Protein SSX3"
}